{
  "gene_symbol": "IQCF5",
  "term_label": "calmodulin binding",
  "gene_name": "IQ domain-containing protein F5",
  "term_id": "GO:0005516",
  "gene": "UniProtKB:A8MTL0"
}